{
  "term_label": "Unknown biological process",
  "gene": "UniProtKB:A0A1B0GU33",
  "term_id": "UNKNOWN:0002",
  "gene_name": "Testis-expressed protein 53",
  "gene_symbol": "TEX53"
}